periplasmic side of plasma membrane [GO:0098567] (cellular component) Definition: The side (leaflet) of a plasma membrane that faces the periplasm, and all proteins embedded in it or attached to its surface. Sources: GOC:dos Relationships: is a type of external side of plasma membrane [GO:0009897]